fructan catabolic process [GO:0010147] (biological process) Also known as: fructan breakdown, fructan catabolism, fructan degradation, levan catabolic process, levan catabolism Relationships: is a type of polysaccharide catabolic process [GO:0000272] Sources: GOC:pz Definition: The chemical reactions and pathways resulting in the breakdown of fructan, a polysaccharide consisting of fructose residues. Subtypes: inulin catabolic process [GO:1902927]